RNA localization to nucleus [GO:0090685] (biological process) Also known as: RNA localisation to nucleus Relationships: is_a RNA localization [GO:0006403] Subtypes: GO:0090670 References: PMID:26305931 Sources: GOC:mah Definition: A macromolecular localization process in which RNA is transported to and maintained in a location within the nucleus.